{
  "term_label": "nucleus",
  "gene": "UniProtKB:Q9UKA9",
  "gene_name": "Polypyrimidine tract-binding protein 2",
  "gene_symbol": "PTBP2",
  "term_id": "GO:0005634"
}